cell cycle DNA replication [GO:0044786] (biological process) Subtypes: nuclear DNA replication [GO:0033260], DNA endoreduplication [GO:0042023], bacterial-type DNA replication [GO:0044787] Sources: GOC:mtg_cell_cycle Definition: The DNA-dependent DNA replication that takes place as part of the cell cycle. Relationships: is a type of GO:0006261; is a type of GO:0022402